{
  "term_label": "neutrophil chemotaxis",
  "gene_name": "High affinity immunoglobulin epsilon receptor subunit gamma",
  "gene": "UniProtKB:P30273",
  "term_id": "GO:0030593",
  "gene_symbol": "FCER1G"
}